{
  "gene_symbol": "PACSIN1",
  "gene": "UniProtKB:Q9BY11",
  "term_label": "cytoplasm",
  "gene_name": "Protein kinase C and casein kinase substrate in neurons protein 1",
  "term_id": "GO:0005737"
}